{
  "gene_name": "DNA excision repair protein ERCC-8",
  "term_id": "UNKNOWN:0001",
  "gene": "UniProtKB:Q13216",
  "gene_symbol": "ERCC8",
  "term_label": "Unknown molecular function"
}